{
  "gene_symbol": "RNF215",
  "term_label": "ubiquitin protein ligase activity",
  "gene": "UniProtKB:Q9Y6U7",
  "gene_name": "RING finger protein 215",
  "term_id": "GO:0061630"
}